{
  "term_label": "cytokine-mediated signaling pathway",
  "gene": "UniProtKB:Q99062",
  "term_id": "GO:0019221",
  "gene_name": "Granulocyte colony-stimulating factor receptor",
  "gene_symbol": "CSF3R"
}